{
  "gene_name": "E3 SUMO-protein ligase ZBED1",
  "gene": "UniProtKB:O96006",
  "term_label": "regulation of transcription by RNA polymerase II",
  "gene_symbol": "ZBED1",
  "term_id": "GO:0006357"
}